positive regulation of protein deacetylation [GO:0090312] (biological process) Also known as: positive regulation of protein amino acid deacetylation Relationships: is_a positive regulation of protein modification process [GO:0031401]; is a type of regulation of protein deacetylation [GO:0090311]; positively regulates GO:0006476 Subtypes: positive regulation of tubulin deacetylation [GO:0090044] Definition: Any process that increases the rate, frequency, or extent of protein deacetylation, the removal of an acetyl group from a protein amino acid. An acetyl group is CH3CO-, derived from acetic [ethanoic] acid. References: PMID:20027304 Sources: GOC:ecd